pyrenoid tubule [GO:0160223] (cellular component) Also known as: thylakoid membrane tubule References: PMID:32428480 Definition: A specialized membranous structure that extends from the photosynthetic thylakoid membrane into and transverses the matrix of a pyrenoid. Relationships: is a type of cellular anatomical structure [GO:0110165]; BFO_0000050 pyrenoid [GO:1990732]